{
  "gene_name": "Trichoplein keratin filament-binding protein",
  "gene": "UniProtKB:Q9BT92",
  "term_id": "GO:0045095",
  "gene_symbol": "TCHP",
  "term_label": "keratin filament"
}